{
  "gene_symbol": "TRIM49B",
  "term_label": "innate immune response",
  "gene": "UniProtKB:A6NDI0",
  "term_id": "GO:0045087",
  "gene_name": "Putative tripartite motif-containing protein 49B"
}